{
  "term_label": "3',5'-cyclic-GMP phosphodiesterase activity",
  "gene": "UniProtKB:Q9NP56",
  "gene_name": "cAMP-specific 3',5'-cyclic phosphodiesterase 7B",
  "term_id": "GO:0047555",
  "gene_symbol": "PDE7B"
}